L-arabitol catabolic process to D-xylulose 5-phosphate [GO:0019590] (biological process) Sources: GOC:curators Relationships: is a type of L-arabitol catabolic process [GO:0051158]; is a type of D-xylulose 5-phosphate metabolic process [GO:0051167] Definition: The chemical reactions and pathways resulting in the breakdown of L-arabitol to form D-xylulose 5-phosphate. L-arabitol is converted into L-xylulose, which is then phosphorylated to L-xylulose-5-phosphate. This is converted to D-xylulose-5-phosphate via the intermediate L-ribulose-5-phosphate. Also known as: L-arabitol and xylitol degradation, L-arabitol breakdown to xylulose 5-phosphate, L-arabitol degradation to xylulose 5-phosphate, L-arabitol utilization